{
  "gene_symbol": "NKX3-2",
  "term_label": "RNA polymerase II cis-regulatory region sequence-specific DNA binding",
  "term_id": "GO:0000978",
  "gene": "UniProtKB:P78367",
  "gene_name": "Homeobox protein Nkx-3.2"
}